mammary gland duct morphogenesis [GO:0060603] (biological process) Definition: The process in which anatomical structures of the mammary ducts are generated and organized. Mammary ducts are epithelial tubes that transport milk. References: PMID:17120154 Sources: GOC:dph Relationships: is a type of GO:0060562; is part of mammary gland morphogenesis [GO:0060443]; is part of mammary gland epithelium development [GO:0061180]